{
  "gene_symbol": "INHBB",
  "term_label": "cytokine activity",
  "gene": "UniProtKB:P09529",
  "term_id": "GO:0005125",
  "gene_name": "Inhibin beta B chain"
}